chondroitin sulfate binding [GO:0035374] (molecular function) Definition: Binding to chondroitin sulfate, a glycosaminoglycan made up of two alternating monosaccharides: D-glucuronic acid (GlcA) and N-acetyl-D-galactosamine (GalNAc). Sources: GOC:kmv, ISBN:0198506732 Relationships: is a type of GO:0005539; is a type of sulfur compound binding [GO:1901681]